axo-dendritic protein transport [GO:0099640] (biological process) Definition: The directed movement of proteins along microtubules in neuron projections. Sources: ISBN:0815316194 Also known as: axonal protein transport Relationships: is a type of axo-dendritic transport [GO:0008088]; is a type of protein transport along microtubule [GO:0098840] Subtypes: anterograde axonal protein transport [GO:0099641], retrograde axonal protein transport [GO:0099642] Regulation: regulated by regulation of axo-dendritic protein transport [GO:1905126]; negatively regulated by negative regulation of axo-dendritic protein transport [GO:1905127]; positively regulated by positive regulation of axo-dendritic protein transport [GO:1905128]